{
  "gene": "UniProtKB:Q15669",
  "gene_name": "Rho-related GTP-binding protein RhoH",
  "term_id": "GO:0007015",
  "term_label": "actin filament organization",
  "gene_symbol": "RHOH"
}